{
  "term_id": "GO:0042995",
  "term_label": "cell projection",
  "gene_symbol": "SPTAN1",
  "gene_name": "Spectrin alpha chain, non-erythrocytic 1",
  "gene": "UniProtKB:Q13813"
}